{
  "gene": "UniProtKB:A0A075B6X9",
  "gene_symbol": "TRAJ18",
  "gene_name": "T cell receptor alpha joining 18 (Fragment)",
  "term_label": "Unknown cellular component",
  "term_id": "UNKNOWN:0003"
}